{
  "term_id": "GO:0030424",
  "term_label": "axon",
  "gene_symbol": "INSR",
  "gene": "UniProtKB:P06213",
  "gene_name": "Insulin receptor"
}